{
  "term_label": "cytoplasm",
  "gene": "UniProtKB:P49327",
  "term_id": "GO:0005737",
  "gene_name": "Fatty acid synthase",
  "gene_symbol": "FASN"
}